{
  "term_id": "GO:0003756",
  "term_label": "protein disulfide isomerase activity",
  "gene_symbol": "PDIA5",
  "gene": "UniProtKB:Q14554",
  "gene_name": "Protein disulfide-isomerase A5"
}